{
  "term_id": "GO:0140693",
  "gene_name": "Cell division cycle-associated protein 2",
  "gene": "UniProtKB:Q69YH5",
  "term_label": "molecular condensate scaffold activity",
  "gene_symbol": "CDCA2"
}